{
  "gene_name": "Heat shock 70 kDa protein 14",
  "gene_symbol": "HSPA14",
  "gene": "UniProtKB:Q0VDF9",
  "term_id": "GO:0005829",
  "term_label": "cytosol"
}